{
  "gene_symbol": "CEP19",
  "term_label": "vesicle targeting, trans-Golgi to periciliary membrane compartment",
  "gene": "UniProtKB:Q96LK0",
  "gene_name": "Centrosomal protein of 19 kDa",
  "term_id": "GO:0097712"
}